{
  "gene": "UniProtKB:Q01780",
  "term_id": "GO:0005730",
  "gene_symbol": "EXOSC10",
  "gene_name": "Exosome component 10",
  "term_label": "nucleolus"
}